ferric-vibriobactin transmembrane transporter activity [GO:0019535] (molecular function) Definition: Enables the transfer of ferric-vibriobactin ions from one side of a membrane to the other. Relationships: is a type of iron chelate transmembrane transporter activity [GO:0015603] Sources: GOC:ai